{
  "gene_name": "Lysosomal acid phosphatase",
  "term_id": "GO:0007040",
  "gene_symbol": "ACP2",
  "gene": "UniProtKB:P11117",
  "term_label": "lysosome organization"
}